{
  "gene_symbol": "MNX1",
  "term_label": "spinal cord motor neuron cell fate specification",
  "term_id": "GO:0021520",
  "gene": "UniProtKB:P50219",
  "gene_name": "Motor neuron and pancreas homeobox protein 1"
}